{
  "gene": "UniProtKB:Q9Y6A1",
  "gene_symbol": "POMT1",
  "term_id": "GO:0035269",
  "gene_name": "Protein O-mannosyl-transferase 1",
  "term_label": "protein O-linked glycosylation via mannose"
}